single fertilization [GO:0007338] (BP) Definition: The union of male and female gametes to form a zygote. Also known as: zygote biosynthesis, zygote formation Relationships: is a type of fertilization [GO:0009566] Sources: GOC:ems, GOC:mtg_sensu